{
  "gene_symbol": "CAMKK1",
  "term_label": "intracellular signal transduction",
  "gene": "UniProtKB:Q8N5S9",
  "term_id": "GO:0035556",
  "gene_name": "Calcium_calmodulin-dependent protein kinase kinase 1"
}